{
  "term_label": "Unknown biological process",
  "term_id": "UNKNOWN:0002",
  "gene_name": "Hippocampus abundant transcript 1 protein",
  "gene": "UniProtKB:Q96MC6",
  "gene_symbol": "MFSD14A"
}